negative regulation of metaphase/anaphase transition of meiosis II [GO:1905190] (biological process) Also known as: negative regulation of meiosis II metaphase/anaphase transition Definition: Any process that stops, prevents or reduces the frequency, rate or extent of metaphase/anaphase transition of meiosis II. References: PMID:21389117 Sources: GOC:TermGenie, GO_REF:0000058 Relationships: is a type of GO:1902103; is a type of GO:1905189; negatively regulates metaphase/anaphase transition of meiosis II [GO:1990950]